positive regulation of chondrocyte development [GO:1902761] (biological process) Also known as: up regulation of chondrocyte development, up-regulation of chondrocyte development, upregulation of chondrocyte development, activation of chondrocyte development References: PMID:16575901 Sources: GOC:TermGenie, GOC:mr, GO_REF:0000058 Definition: Any process that activates or increases the frequency, rate or extent of chondrocyte development. Relationships: is a type of positive regulation of cell development [GO:0010720]; is a type of positive regulation of chondrocyte differentiation [GO:0032332]; is a type of regulation of chondrocyte development [GO:0061181]; positively regulates GO:0002063 Subtypes: GO:1903043